{
  "gene": "UniProtKB:P08133",
  "gene_name": "Annexin A6",
  "term_label": "cytoplasm",
  "term_id": "GO:0005737",
  "gene_symbol": "ANXA6"
}